cytokinin receptor activity [GO:0009884] (molecular function) Sources: GOC:lr, GOC:signaling Relationships: is a type of transmembrane signaling receptor activity [GO:0004888]; is part of GO:0009736 Subtypes: G protein-coupled cytokinin receptor activity [GO:0001647], transmembrane histidine kinase cytokinin receptor activity [GO:0009885] Definition: Combining with a cytokinin and transmitting the signal from one side of the membrane to the other to initiate a change in cell activity.